{
  "gene_name": "Putative upstream-binding factor 1-like protein 6",
  "gene_symbol": "UBTFL6",
  "gene": "UniProtKB:P0CB48",
  "term_id": "GO:0045943",
  "term_label": "positive regulation of transcription by RNA polymerase I"
}